{
  "gene": "UniProtKB:Q9GZZ9",
  "gene_symbol": "UBA5",
  "term_label": "cytosol",
  "gene_name": "Ubiquitin-like modifier-activating enzyme 5",
  "term_id": "GO:0005829"
}